{
  "term_id": "GO:0140312",
  "term_label": "cargo adaptor activity",
  "gene_symbol": "COG3",
  "gene": "UniProtKB:Q96JB2",
  "gene_name": "Conserved oligomeric Golgi complex subunit 3"
}